{
  "gene_symbol": "AVIL",
  "term_id": "GO:0051016",
  "gene_name": "Advillin",
  "gene": "UniProtKB:O75366",
  "term_label": "barbed-end actin filament capping"
}